{
  "gene_symbol": "TRMT2B",
  "gene": "UniProtKB:Q96GJ1",
  "term_id": "UNKNOWN:0002",
  "gene_name": "tRNA (uracil-5-)-methyltransferase homolog B",
  "term_label": "Unknown biological process"
}